gluconeogenesis [GO:0006094] (biological process) Sources: MetaCyc:GLUCONEO-PWY Definition: The formation of glucose from noncarbohydrate precursors, such as pyruvate, amino acids and glycerol. Relationships: is a type of glucose metabolic process [GO:0006006]; is a type of hexose biosynthetic process [GO:0019319] Regulation: RO_0002211 by regulation of gluconeogenesis [GO:0006111]; negatively regulated by negative regulation of gluconeogenesis [GO:0045721]; positively regulated by positive regulation of gluconeogenesis [GO:0045722] Also known as: glucose biosynthesis, glucose biosynthetic process